{
  "term_label": "neuron projection",
  "term_id": "GO:0043005",
  "gene_name": "Disks large homolog 3",
  "gene_symbol": "DLG3",
  "gene": "UniProtKB:Q92796"
}